{
  "term_id": "GO:0005634",
  "gene": "UniProtKB:Q9UDT6",
  "gene_symbol": "CLIP2",
  "term_label": "nucleus",
  "gene_name": "CAP-Gly domain-containing linker protein 2"
}